{
  "term_label": "aspartic-type endopeptidase activity",
  "term_id": "GO:0004190",
  "gene_name": "Beta-secretase 1",
  "gene_symbol": "BACE1",
  "gene": "UniProtKB:P56817"
}